chloroplast localization [GO:0019750] (biological process) Also known as: chloroplast localisation Subtypes: chloroplast relocation [GO:0009902] Relationships: is a type of plastid localization [GO:0051644] Sources: GOC:bf, GOC:jl, ISBN:0198506732 Definition: Any process in which a chloroplast is transported to, and/or maintained in, a specific location within the cell. A chloroplast is a chlorophyll-containing plastid found in cells of algae and higher plants.